{
  "gene_symbol": "ZKSCAN4",
  "gene": "UniProtKB:Q969J2",
  "term_id": "GO:0000981",
  "term_label": "DNA-binding transcription factor activity, RNA polymerase II-specific",
  "gene_name": "Zinc finger protein with KRAB and SCAN domains 4"
}